{
  "gene_name": "UDP-N-acetylhexosamine pyrophosphorylase-like protein 1",
  "term_label": "UDP-N-acetylglucosamine diphosphorylase activity",
  "gene_symbol": "UAP1L1",
  "gene": "UniProtKB:Q3KQV9",
  "term_id": "GO:0003977"
}